{
  "term_id": "GO:0061630",
  "gene_symbol": "SIAH3",
  "gene_name": "Seven in absentia homolog 3",
  "term_label": "ubiquitin protein ligase activity",
  "gene": "UniProtKB:Q8IW03"
}